{
  "gene_symbol": "DERL2",
  "gene": "UniProtKB:Q9GZP9",
  "gene_name": "Derlin-2",
  "term_id": "GO:0036503",
  "term_label": "ERAD pathway"
}